{
  "gene_name": "Hemoglobin subunit theta-1",
  "gene_symbol": "HBQ1",
  "gene": "UniProtKB:P09105",
  "term_label": "oxygen carrier activity",
  "term_id": "GO:0005344"
}